{
  "term_id": "GO:0061630",
  "gene_name": "Probable E3 ubiquitin-protein ligase DTX2",
  "term_label": "ubiquitin protein ligase activity",
  "gene": "UniProtKB:Q86UW9",
  "gene_symbol": "DTX2"
}